{
  "gene": "UniProtKB:Q96BQ1",
  "gene_name": "Protein FAM3D",
  "term_id": "GO:0007165",
  "gene_symbol": "FAM3D",
  "term_label": "signal transduction"
}